{
  "gene": "UniProtKB:P36402",
  "term_label": "regulation of transcription by RNA polymerase II",
  "term_id": "GO:0006357",
  "gene_symbol": "TCF7",
  "gene_name": "Transcription factor 7"
}